cellular response to L-thialysine [GO:0072751] (biological process) Also known as: cellular response to thialysine Relationships: is a type of cellular response to amino acid stimulus [GO:0071230]; is a type of response to L-thialysine [GO:1901345]; is a type of cellular response to nitrogen compound [GO:1901699]; is a type of cellular response to oxygen-containing compound [GO:1901701] Sources: GOC:mah Definition: Any process that results in a change in state or activity of a cell (in terms of movement, secretion, enzyme production, gene expression, etc.) as a result of a L-thialysine stimulus.